{
  "gene": "UniProtKB:Q9H2V7",
  "term_id": "GO:0016020",
  "gene_name": "Protein spinster homolog 1",
  "gene_symbol": "SPNS1",
  "term_label": "membrane"
}